{
  "gene_name": "Protein THEMIS",
  "term_label": "nucleus",
  "gene_symbol": "THEMIS",
  "gene": "UniProtKB:Q8N1K5",
  "term_id": "GO:0005634"
}